{
  "gene_name": "Protocadherin-15",
  "term_id": "GO:0045202",
  "gene_symbol": "PCDH15",
  "gene": "UniProtKB:Q96QU1",
  "term_label": "synapse"
}